{
  "gene_symbol": "ATP8A1",
  "gene": "UniProtKB:Q9Y2Q0",
  "term_id": "GO:0140326",
  "gene_name": "Phospholipid-transporting ATPase IA",
  "term_label": "ATPase-coupled intramembrane lipid transporter activity"
}